replication inhibiting complex [GO:1990078] (cellular component) Subtypes: DnaA-L2 complex [GO:1990082], DnaA-Hda complex [GO:1990083], GO:1990084, Hda-beta clamp complex [GO:1990085] Definition: A protein complex that inhibits multiple events of replication initiation during one replication cycle. Relationships: is a type of protein-containing complex [GO:0032991]; is part of replisome [GO:0030894] References: PMID:21708944 Sources: GOC:bhm